{
  "gene": "UniProtKB:Q9H1Z8",
  "gene_name": "Augurin",
  "gene_symbol": "ECRG4",
  "term_label": "central nervous system development",
  "term_id": "GO:0007417"
}